{
  "term_label": "G protein-coupled receptor activity",
  "gene_symbol": "CMKLR1",
  "gene_name": "Chemerin-like receptor 1",
  "gene": "UniProtKB:Q99788",
  "term_id": "GO:0004930"
}